{
  "term_label": "cytokine binding",
  "gene_symbol": "CRLF1",
  "term_id": "GO:0019955",
  "gene": "UniProtKB:O75462",
  "gene_name": "Cytokine receptor-like factor 1"
}